positive regulation of systemic acquired resistance [GO:1901672] (biological process) Sources: GOC:TermGenie Also known as: activation of salicylic acid-dependent systemic resistance, positive regulation of salicylic acid-dependent systemic resistance, up regulation of salicylic acid-dependent systemic resistance, up regulation of systemic acquired resistance, up-regulation of salicylic acid-dependent systemic resistance, up-regulation of systemic acquired resistance, upregulation of salicylic acid-dependent systemic resistance, upregulation of systemic acquired resistance, activation of systemic acquired resistance Definition: Any process that activates or increases the frequency, rate or extent of systemic acquired resistance. Relationships: is a type of positive regulation of response to biotic stimulus [GO:0002833]; is a type of regulation of systemic acquired resistance [GO:0010112]; is a type of GO:0031349; is a type of positive regulation of response to external stimulus [GO:0032103]; positively regulates systemic acquired resistance [GO:0009627]